{
  "term_id": "UNKNOWN:0003",
  "term_label": "Unknown cellular component",
  "gene_symbol": "GOLGA6L9",
  "gene_name": "Golgin subfamily A member 6-like protein 9",
  "gene": "UniProtKB:A6NEM1"
}